{
  "gene_name": "Olfactory receptor 10W1",
  "term_label": "Unknown cellular component",
  "term_id": "UNKNOWN:0003",
  "gene": "UniProtKB:Q8NGF6",
  "gene_symbol": "OR10W1"
}